{
  "term_label": "cell development",
  "gene_name": "Iroquois-class homeodomain protein IRX-5",
  "gene_symbol": "IRX5",
  "term_id": "GO:0048468",
  "gene": "UniProtKB:P78411"
}